cyclic-guanylate-specific phosphodiesterase activity [GO:0071111] (MF) Definition: Catalysis of the reaction: cyclic di-3',5'-guanylate + H2O = 5'-phosphoguanylyl(3'->5')guanosine + H+. Sources: EC:3.1.4.52, RHEA:24902 Also known as: PDEA1, VieA, c-di-GMP phosphodiesterase activity, c-di-GMP-specific phosphodiesterase activity, cyclic bis(3->5')diguanylate phosphodiesterase activity, phosphodiesterase A1 activity Relationships: is a type of GO:0008081